{
  "gene_name": "Putative uncharacterized protein ENSP00000347057",
  "gene_symbol": "A6NHS1",
  "gene": "UniProtKB:A6NHS1",
  "term_label": "Unknown biological process",
  "term_id": "UNKNOWN:0002"
}